lateral line nerve glial cell migration [GO:0048896] (biological process) Definition: The movement of a glial cell along the axons in a lateral line nerve. References: PMID:12062041 Also known as: glial cell migration in lateral line nerve Relationships: is a type of glial cell migration [GO:0008347]; is part of lateral line nerve development [GO:0048892] Subtypes: GO:0048912, glial cell migration in posterior lateral line nerve [GO:0048930]